{
  "gene_name": "E3 ubiquitin-protein ligase TRIP12",
  "term_label": "DNA damage response",
  "term_id": "GO:0006974",
  "gene": "UniProtKB:Q14669",
  "gene_symbol": "TRIP12"
}